{
  "gene_name": "Class A basic helix-loop-helix protein 9",
  "gene": "UniProtKB:Q7RTU4",
  "term_id": "GO:0032502",
  "gene_symbol": "BHLHA9",
  "term_label": "developmental process"
}